calcium import into the mitochondrion involved in negative regulation of presynaptic cytosolic calcium concentration [GO:1905743] (biological process) Relationships: is a type of GO:0036444; is a type of GO:0051649; is part of negative regulation of presynaptic cytosolic calcium concentration [GO:0099113] Also known as: calcium ion transmembrane import into mitochondrion involved in negative regulation of presynaptic cytosolic calcium concentration, mitochondrial calcium uptake involved in negative regulation of presynaptic cytosolic calcium concentration References: PMID:26644474 Sources: GOC:TermGenie, GO_REF:0000060 Definition: Any mitochondrial calcium uptake that is involved in negative regulation of presynaptic cytosolic calcium concentration.